{
  "gene_name": "Cystatin-9-like",
  "term_label": "extracellular space",
  "gene": "UniProtKB:Q9H4G1",
  "gene_symbol": "CST9L",
  "term_id": "GO:0005615"
}